monocarboxylic acid biosynthetic process [GO:0072330] (BP) Also known as: monocarboxylic acid anabolism, monocarboxylic acid biosynthesis, monocarboxylic acid formation, monocarboxylic acid synthesis Relationships: is a type of GO:0032787; is a type of GO:0046394 Subtypes: retinoic acid biosynthetic process [GO:0002138], creatine biosynthetic process [GO:0006601], fatty acid biosynthetic process [GO:0006633], GO:0006699, GO:0008153, biotin biosynthetic process [GO:0009102], indoleacetic acid biosynthetic process [GO:0009684], GO:0009688, GO:0009697, cinnamic acid biosynthetic process [GO:0009800], GO:0010379, pantothenate biosynthetic process [GO:0015940], formate biosynthetic process [GO:0015943], lactate biosynthetic process [GO:0019249], coenzyme B biosynthetic process [GO:0019298], acetate biosynthetic process [GO:0019413], GO:0019491, (R)-mandelate catabolic process to benzoate [GO:0019597], GO:0033050, GO:0033481, ferulate biosynthetic process [GO:0033495], sinapate biosynthetic process [GO:0033497], GO:0034276, quinate biosynthetic process [GO:0042194], penicillin biosynthetic process [GO:0042318], pyruvate biosynthetic process [GO:0042866], aldonic acid biosynthetic process [GO:0046175], mandelate biosynthetic process [GO:0046236], GO:0046277, GO:0046279, GO:0046295, GO:0046399, L-pipecolic acid biosynthetic process [GO:0062034], mycophenolic acid biosynthetic process [GO:0140722], o-orsellinic acid biosynthetic process [GO:1900584], ochratoxin A biosynthetic process [GO:1900818], GO:1901024, 2-dehydro-3-deoxy-D-gluconic acid biosynthetic process [GO:1901274], cyclic 2,3-bisphospho-D-glycerate biosynthetic process [GO:1901369], olivetolic acid biosynthetic process [GO:1901697], (R)-mevalonic acid biosynthetic process [GO:1901737], pentalenolactone biosynthetic process [GO:1901780], p-cumate biosynthetic process [GO:1901783], 3-(2,3-dihydroxyphenyl)propanoate biosynthetic process [GO:1901792], GO:1901795, nicotinate biosynthetic process [GO:1901849], fumagillin biosynthetic process [GO:1902086], glycyrrhetinate biosynthetic process [GO:1902386], picolinic acid biosynthetic process [GO:1905004] Definition: The chemical reactions and pathways resulting in the formation of monocarboxylic acids, any organic acid containing one carboxyl (-COOH) group. Sources: GOC:mah